oocyte microtubule cytoskeleton organization [GO:0016325] (biological process) Also known as: oocyte microtubule cytoskeleton organisation Definition: Formation and maintenance of a polarized microtubule array originating from a microtubule-organizing center (MTOC) in the oocyte. An example of this is found in Drosophila melanogaster. References: PMID:11231123 Sources: GOC:mtg_sensu Relationships: is a type of GO:0030951; is part of GO:0007308